{
  "term_label": "cytoplasm",
  "gene_name": "Myosin light chain kinase 3",
  "gene_symbol": "MYLK3",
  "term_id": "GO:0005737",
  "gene": "UniProtKB:Q32MK0"
}